asparagine transmembrane transport [GO:1903713] (biological process) Definition: The directed movement of asparagine across a membrane. References: PMID:18503766 Sources: GOC:TermGenie, GO_REF:0000069 Relationships: is a type of amino acid transmembrane transport [GO:0003333]; is_a amide transport [GO:0042886]; is a type of carboxylic acid transmembrane transport [GO:1905039] Subtypes: L-asparagine import across plasma membrane [GO:1903811], asparagine transmembrane import into vacuole [GO:1990591]